{
  "gene_symbol": "CEACAM7",
  "gene": "UniProtKB:Q14002",
  "gene_name": "Carcinoembryonic antigen-related cell adhesion molecule 7",
  "term_label": "regulation of immune system process",
  "term_id": "GO:0002682"
}